{
  "gene": "UniProtKB:Q8TD17",
  "gene_name": "Zinc finger protein 398",
  "term_label": "nucleus",
  "gene_symbol": "ZNF398",
  "term_id": "GO:0005634"
}